{
  "term_label": "glutamate decarboxylase activity",
  "gene_name": "Glutamate decarboxylase 2",
  "term_id": "GO:0004351",
  "gene_symbol": "GAD2",
  "gene": "UniProtKB:Q05329"
}